{
  "gene_symbol": "TEX22",
  "gene": "UniProtKB:C9J3V5",
  "gene_name": "Testis-expressed protein 22",
  "term_label": "Unknown biological process",
  "term_id": "UNKNOWN:0002"
}